positive regulation of beta-catenin-TCF complex assembly [GO:1904865] (BP) Definition: Any process that activates or increases the frequency, rate or extent of beta-catenin-TCF complex assembly. Also known as: positive regulation of beta-catenin-TCF complex formation, up regulation of beta-catenin-TCF complex assembly, up regulation of beta-catenin-TCF complex formation, up-regulation of beta-catenin-TCF complex assembly, up-regulation of beta-catenin-TCF complex formation, upregulation of beta-catenin-TCF complex assembly, upregulation of beta-catenin-TCF complex formation, activation of beta-catenin-TCF complex assembly, activation of beta-catenin-TCF complex formation, activation of beta-catenin/LEF complex assembly, activation of beta-catenin/LEF complex formation, positive regulation of beta-catenin/LEF complex assembly, positive regulation of beta-catenin/LEF complex formation, up regulation of beta-catenin/LEF complex assembly, up regulation of beta-catenin/LEF complex formation, up-regulation of beta-catenin/LEF complex assembly, up-regulation of beta-catenin/LEF complex formation, upregulation of beta-catenin/LEF complex assembly, upregulation of beta-catenin/LEF complex formation, activation of beta-catenin/T-cell factor complex assembly, activation of beta-catenin/T-cell factor complex formation, activation of beta-catenin/lymphoid enhancer binding factor complex assembly, activation of beta-catenin/lymphoid enhancer binding factor complex formation, positive regulation of beta-catenin/T-cell factor complex assembly, positive regulation of beta-catenin/T-cell factor complex formation, positive regulation of beta-catenin/lymphoid enhancer binding factor complex assembly, positive regulation of beta-catenin/lymphoid enhancer binding factor complex formation, up regulation of beta-catenin/T-cell factor complex assembly, up regulation of beta-catenin/T-cell factor complex formation, up regulation of beta-catenin/lymphoid enhancer binding factor complex assembly, up regulation of beta-catenin/lymphoid enhancer binding factor complex formation, up-regulation of beta-catenin/T-cell factor complex assembly, up-regulation of beta-catenin/T-cell factor complex formation, up-regulation of beta-catenin/lymphoid enhancer binding factor complex assembly, up-regulation of beta-catenin/lymphoid enhancer binding factor complex formation, upregulation of beta-catenin/T-cell factor complex assembly, upregulation of beta-catenin/T-cell factor complex formation, upregulation of beta-catenin/lymphoid enhancer binding factor complex assembly, upregulation of beta-catenin/lymphoid enhancer binding factor complex formation Relationships: is a type of positive regulation of protein-containing complex assembly [GO:0031334]; is a type of regulation of beta-catenin-TCF complex assembly [GO:1904863]; positively regulates beta-catenin-TCF complex assembly [GO:1904837] Sources: GOC:PARL, GOC:TermGenie, GOC:bf, GO_REF:0000058